{
  "gene_symbol": "NT5M",
  "term_id": "GO:0008253",
  "gene_name": "5'(3')-deoxyribonucleotidase, mitochondrial",
  "term_label": "5'-nucleotidase activity",
  "gene": "UniProtKB:Q9NPB1"
}